negative regulation of flocculation [GO:0060257] (biological process) Also known as: negative regulation of coflocculation Definition: Any process that decreases the rate, frequency or extent of the non-sexual aggregation of single-celled organisms. Sources: GOC:dph, GOC:tb Relationships: is a type of GO:0022408; is a type of regulation of flocculation [GO:0060256]; negatively regulates flocculation [GO:0000128]